regulation of leukocyte mediated cytotoxicity [GO:0001910] (biological process) Also known as: regulation of immune cell mediated cell death, regulation of immune cell mediated cell killing, regulation of immune cell mediated cytotoxicity, regulation of leucocyte mediated cytotoxicity Subtypes: regulation of antibody-dependent cellular cytotoxicity [GO:0001813], negative regulation of leukocyte mediated cytotoxicity [GO:0001911], GO:0001912, regulation of T cell mediated cytotoxicity [GO:0001914], GO:0042269, regulation of neutrophil mediated cytotoxicity [GO:0070948], regulation of microglial cell mediated cytotoxicity [GO:1904149] References: PMID:11911826 Sources: GOC:add, ISBN:0781735149 Definition: Any process that modulates the frequency, rate, or extent of leukocyte mediated cytotoxicity. Relationships: is a type of regulation of leukocyte mediated immunity [GO:0002703]; is a type of GO:0031341; regulates GO:0001909